{
  "term_id": "GO:0005737",
  "gene_name": "Probable ATP-dependent RNA helicase DDX5",
  "term_label": "cytoplasm",
  "gene": "UniProtKB:P17844",
  "gene_symbol": "DDX5"
}